{
  "gene_name": "Kunitz-type protease inhibitor 2",
  "term_label": "serine-type endopeptidase inhibitor activity",
  "gene_symbol": "SPINT2",
  "gene": "UniProtKB:O43291",
  "term_id": "GO:0004867"
}